AIM2 inflammasome complex [GO:0097169] (cellular component) Relationships: is a type of GO:0061702 Definition: An inflammasome complex that consists of AIM2, ASC, and caspase-1. AIM2 is a member of the HN-200 protein family that appears to be the sensor of cytosolic double-stranded DNA. References: PMID:20303873 Sources: GOC:vp